{
  "gene_symbol": "TTC17",
  "gene_name": "Tetratricopeptide repeat protein 17",
  "gene": "UniProtKB:Q96AE7",
  "term_label": "actin cytoskeleton",
  "term_id": "GO:0015629"
}